{
  "term_label": "regulation of gene expression",
  "gene_symbol": "TRIM49B",
  "gene_name": "Putative tripartite motif-containing protein 49B",
  "gene": "UniProtKB:A6NDI0",
  "term_id": "GO:0010468"
}